classical arabinogalactan protein metabolic process [GO:0010406] (biological process) Relationships: is a type of arabinogalactan protein metabolic process [GO:0010405] Sources: GOC:tair_curators Definition: The chemical reactions and pathways involving a cell wall arabinogalactan II glycoprotein, which is composed of a group of core protein containing Hyp, Ala, Ser, Thr and Gly as the major amino acid constituents, and the C-terminus is GPI anchored. Also known as: classical-arabinogalactan protein metabolism